{
  "gene": "UniProtKB:Q8NDL9",
  "gene_name": "Cytosolic carboxypeptidase-like protein 5",
  "term_label": "Unknown biological process",
  "term_id": "UNKNOWN:0002",
  "gene_symbol": "AGBL5"
}